monoubiquitinated protein deubiquitination [GO:0035520] (biological process) Sources: GOC:bf Definition: The removal of the ubiquitin group from a monoubiquitinated protein. Relationships: is a type of GO:0016579 Also known as: monoubiquitinated protein deubiquitinylation, monoubiquitinated protein deubiquitylation